{
  "gene_symbol": "CALD1",
  "gene_name": "Caldesmon",
  "gene": "UniProtKB:Q05682",
  "term_label": "actin filament bundle assembly",
  "term_id": "GO:0051017"
}